positive regulation of steroid hormone secretion [GO:2000833] (biological process) Subtypes: positive regulation of ecdysteroid secretion [GO:0046000], positive regulation of androgen secretion [GO:2000836], positive regulation of corticosteroid hormone secretion [GO:2000848], positive regulation of estrogen secretion [GO:2000863], positive regulation of estradiol secretion [GO:2000866], positive regulation of estrone secretion [GO:2000869], positive regulation of progesterone secretion [GO:2000872] Definition: Any process that activates or increases the frequency, rate or extent of steroid hormone secretion. Relationships: is a type of positive regulation of lipid transport [GO:0032370]; is a type of positive regulation of hormone secretion [GO:0046887]; is a type of positive regulation of multicellular organismal process [GO:0051240]; is a type of regulation of steroid hormone secretion [GO:2000831]; RO_0002213 steroid hormone secretion [GO:0035929] Sources: GOC:sl